{
  "gene_symbol": "CALCOCO1",
  "term_id": "GO:0003713",
  "term_label": "transcription coactivator activity",
  "gene_name": "Calcium-binding and coiled-coil domain-containing protein 1",
  "gene": "UniProtKB:Q9P1Z2"
}